{
  "term_label": "nuclear envelope",
  "term_id": "GO:0005635",
  "gene_name": "Importin-9",
  "gene_symbol": "IPO9",
  "gene": "UniProtKB:Q96P70"
}